toxin catabolic process [GO:0009407] (biological process) Relationships: is a type of catabolic process [GO:0009056]; is a type of toxin metabolic process [GO:0009404]; is a type of GO:0098754 Sources: GOC:go_curators Also known as: toxin breakdown, toxin catabolism, toxin degradation Subtypes: mycotoxin catabolic process [GO:0043387], sterigmatocystin catabolic process [GO:0045574], bacteriocin catabolic process [GO:0046225], insecticide catabolic process [GO:0046701], phytoalexin catabolic process [GO:0052316] Definition: The chemical reactions and pathways resulting in the breakdown of toxin, a poisonous compound (typically a protein) that is produced by cells or organisms and that can cause disease when introduced into the body or tissues of an organism.